2-deoxystreptamine biosynthetic process [GO:1901744] (biological process) Sources: GOC:TermGenie, GOC:yaf, UniPathway:UPA00907 Definition: The chemical reactions and pathways resulting in the formation of 2-deoxystreptamine. Also known as: 2-deoxystreptamine anabolism, 2-deoxystreptamine biosynthesis, 2-deoxystreptamine formation, 2-deoxystreptamine synthesis Relationships: is a type of polyol biosynthetic process [GO:0046173]; is a type of 2-deoxystreptamine metabolic process [GO:1901742]